prothoracicotrophic hormone activity [GO:0018445] (molecular function) Relationships: is a type of GO:0005184 References: PMID:3301403 Sources: GOC:mah Definition: The action characteristic of prothoracicotrophic hormone, a peptide hormone that is secreted by the brain and, upon receptor binding, acts on the prothoracic gland to stimulate the release of ecdysone in insects.